UDP-N-acetylgalactosamine transmembrane transport [GO:0015789] (biological process) Sources: GOC:ai Relationships: is a type of GO:0015711; is_a pyrimidine nucleotide-sugar transmembrane transport [GO:0090481] Definition: The directed movement of UDP-N-acetylgalactosamine into, out of or within a cell, or between cells, by means of some agent such as a transporter or pore. UDP-N-acetylgalactosamine is a substance composed of N-acetylgalactosamine, a common structural unit of oligosaccharides, in glycosidic linkage with uridine diphosphate. Also known as: UDP-N-acetylgalactosamine transport